{
  "gene": "UniProtKB:Q7L5L3",
  "gene_name": "Lysophospholipase D GDPD3",
  "gene_symbol": "GDPD3",
  "term_label": "phosphoric diester hydrolase activity",
  "term_id": "GO:0008081"
}